{
  "gene_symbol": "ZNF468",
  "gene": "UniProtKB:Q5VIY5",
  "gene_name": "Zinc finger protein 468",
  "term_id": "GO:0006357",
  "term_label": "regulation of transcription by RNA polymerase II"
}